{
  "gene_name": "Vascular endothelial growth factor C",
  "gene": "UniProtKB:P49767",
  "gene_symbol": "VEGFC",
  "term_label": "extracellular space",
  "term_id": "GO:0005615"
}